{
  "gene_name": "FAS-associated factor 2",
  "gene_symbol": "FAF2",
  "term_id": "GO:0036503",
  "gene": "UniProtKB:Q96CS3",
  "term_label": "ERAD pathway"
}